{
  "gene": "UniProtKB:Q9Y6N5",
  "gene_symbol": "SQOR",
  "term_label": "mitochondrion",
  "gene_name": "Sulfide:quinone oxidoreductase, mitochondrial",
  "term_id": "GO:0005739"
}